{
  "term_label": "signal transduction",
  "gene_symbol": "RND3",
  "term_id": "GO:0007165",
  "gene": "UniProtKB:P61587",
  "gene_name": "Rho-related GTP-binding protein RhoE"
}